calcium-independent phospholipase A2 activity [GO:0047499] (molecular function) Definition: Catalysis of the reaction: phosphatidylcholine + H2O = 1-acylglycerophosphocholine + a carboxylate. This reaction does not require Ca2+. References: PMID:34831185 Relationships: is a type of phospholipase A2 activity [GO:0004623] Also known as: calcium-independent cytosolic phospholipase A2 activity